{
  "term_id": "UNKNOWN:0002",
  "gene": "UniProtKB:I3L273",
  "gene_name": "Golgi-associated olfactory signaling regulator",
  "term_label": "Unknown biological process",
  "gene_symbol": "GFY"
}